(-)-pinoresinol metabolic process [GO:1901598] (biological process) Subtypes: (-)-pinoresinol biosynthetic process [GO:1901599], GO:1902123 Sources: GOC:TermGenie Relationships: is a type of GO:0009806; is a type of phenol-containing compound metabolic process [GO:0018958]; is a type of benzene-containing compound metabolic process [GO:0042537] Definition: The chemical reactions and pathways involving (-)-pinoresinol. Also known as: (-)-pinoresinol metabolism